{
  "gene": "UniProtKB:Q9BQB4",
  "term_id": "GO:0036122",
  "gene_name": "Sclerostin",
  "term_label": "BMP binding",
  "gene_symbol": "SOST"
}